{
  "term_label": "Ctf18 RFC-like complex",
  "gene_symbol": "DSCC1",
  "gene_name": "Sister chromatid cohesion protein DCC1",
  "term_id": "GO:0031390",
  "gene": "UniProtKB:Q9BVC3"
}